putrescine:ornithine antiporter activity [GO:0015496] (molecular function) Also known as: putrescine-ornithine antiporter activity, putrescine/ornithine antiporter activity, putrescine:hydrogen symporter activity Relationships: is a type of L-ornithine transmembrane transporter activity [GO:0000064]; is a type of antiporter activity [GO:0015297]; is a type of GO:0015489 Definition: Enables the transfer of a solute or solutes from one side of a membrane to the other according to the reaction: putrescine(out) + ornithine(in) = putrescine(in) + ornithine(out). Sources: TC:2.A.3.2.1